nuclear membrane fusion involved in karyogamy [GO:0048288] (biological process) Also known as: nuclear membrane fusion during karyogamy Relationships: is a type of nuclear membrane fusion [GO:0000740]; is part of GO:0000741 Definition: The joining of 2 or more lipid bilayer membranes that surround the nucleus during the creation of a single nucleus from multiple nuclei. Sources: GOC:jid